negative regulation of ribosomal protein gene transcription from RNA polymerase II promoter in response to nutrient levels [GO:0010691] (biological process) Definition: Any process that decreases the frequency, rate or extent of the synthesis of RNA from ribosomal protein genes by RNA polymerase II, originating at an RNA polymerase II promoter, as a result of a stimulus reflecting the presence, absence, or concentration of nutrients. Relationships: is a type of negative regulation of ribosomal protein gene transcription by RNA polymerase II [GO:0010688]; is a type of cellular response to nutrient levels [GO:0031669] Sources: GOC:dph, GOC:tb, GOC:txnOH